regulation of systemic arterial blood pressure by capillary fluid shift [GO:0003049] (biological process) Definition: The intrinsic circulatory process resulting from capillary fluid shift that modulates the force with which blood travels through the systemic arterial circulatory system. Capillary fluid shift is the movement of fluid across the capillary membrane between the blood and the interstitial fluid compartment. Sources: GOC:mtg_cardio, ISBN:0721643949 Also known as: blood pressure regulation by capillary fluid shift Relationships: is a type of regulation of systemic arterial blood pressure by physical factors [GO:0003045]